{
  "gene_symbol": "PIK3C3",
  "term_id": "GO:0005777",
  "term_label": "peroxisome",
  "gene_name": "Phosphatidylinositol 3-kinase catalytic subunit type 3",
  "gene": "UniProtKB:Q8NEB9"
}